{
  "gene_symbol": "ADAM30",
  "gene_name": "Disintegrin and metalloproteinase domain-containing protein 30",
  "term_id": "GO:0004222",
  "gene": "UniProtKB:Q9UKF2",
  "term_label": "metalloendopeptidase activity"
}